1-phosphatidylinositol-5-kinase activity [GO:0052810] (molecular function) Definition: Catalysis of the reaction: a 1-phosphatidyl-1D-myo-inositol + ATP = a 1-phosphatidyl-1D-myo-inositol 5-phosphate + ADP + H+. Also known as: 1-phosphatidylinositol 5-kinase activity Relationships: is a type of phosphatidylinositol kinase activity [GO:0052742] References: PMID:12270933, PMID:9660759 Sources: RHEA:44680